{
  "term_label": "histone pre-mRNA 3'end processing complex",
  "term_id": "GO:0071204",
  "gene_name": "Histone RNA hairpin-binding protein",
  "gene": "UniProtKB:Q14493",
  "gene_symbol": "SLBP"
}